{
  "gene_symbol": "CHRNA4",
  "term_id": "GO:0034220",
  "term_label": "monoatomic ion transmembrane transport",
  "gene": "UniProtKB:P43681",
  "gene_name": "Neuronal acetylcholine receptor subunit alpha-4"
}